rhythmic excitation [GO:0043179] (biological process) Sources: GOC:go_curators, ISBN:0195088433 Definition: Any process involved in the generation of rhythmic, synchronous excitatory synaptic inputs in a neural circuit. Relationships: is a type of rhythmic synaptic transmission [GO:0060024]